{
  "gene_name": "C-C motif chemokine 23",
  "term_label": "inflammatory response",
  "gene_symbol": "CCL23",
  "term_id": "GO:0006954",
  "gene": "UniProtKB:P55773"
}